negative regulation of synaptic vesicle clustering [GO:2000808] (biological process) Relationships: is a type of negative regulation of transport [GO:0051051]; is a type of regulation of synaptic vesicle clustering [GO:2000807]; negatively regulates synaptic vesicle clustering [GO:0097091] References: PMID:21513708 Definition: Any process that stops, prevents or reduces the frequency, rate or extent of synaptic vesicle clustering.